{
  "term_label": "Unknown cellular component",
  "term_id": "UNKNOWN:0003",
  "gene": "UniProtKB:O15304",
  "gene_symbol": "SIVA1",
  "gene_name": "Apoptosis regulatory protein Siva"
}